{
  "gene_name": "PDZ domain-containing protein 2",
  "gene_symbol": "PDZD2",
  "term_id": "UNKNOWN:0003",
  "gene": "UniProtKB:O15018",
  "term_label": "Unknown cellular component"
}